{
  "term_id": "GO:0000122",
  "gene": "UniProtKB:P41134",
  "gene_name": "DNA-binding protein inhibitor ID-1",
  "term_label": "negative regulation of transcription by RNA polymerase II",
  "gene_symbol": "ID1"
}